{
  "term_label": "Unknown molecular function",
  "gene_name": "V-set and transmembrane domain-containing protein 5",
  "term_id": "UNKNOWN:0001",
  "gene": "UniProtKB:A8MXK1",
  "gene_symbol": "VSTM5"
}